{
  "gene_name": "Pericentriolar material 1 protein",
  "gene": "UniProtKB:Q15154",
  "gene_symbol": "PCM1",
  "term_id": "GO:0034454",
  "term_label": "microtubule anchoring at centrosome"
}